{
  "gene_symbol": "CAPZA3",
  "term_label": "cortical cytoskeleton",
  "gene": "UniProtKB:Q96KX2",
  "term_id": "GO:0030863",
  "gene_name": "F-actin-capping protein subunit alpha-3"
}